{
  "term_id": "GO:0007623",
  "term_label": "circadian rhythm",
  "gene_name": "RNA-binding protein 4B",
  "gene_symbol": "RBM4B",
  "gene": "UniProtKB:Q9BQ04"
}